regulation of presynaptic membrane organization [GO:1901629] (biological process) Definition: Any process that modulates the frequency, rate or extent of presynaptic membrane organization. Subtypes: negative regulation of presynaptic membrane organization [GO:1901630], GO:1901631 Also known as: regulation of pre-synaptic membrane organization, regulation of presynaptic membrane organisation Relationships: is a type of GO:0050807; regulates presynaptic membrane organization [GO:0097090] References: PMID:22426000 Sources: GOC:TermGenie